{
  "gene_symbol": "TKFC",
  "term_label": "glycerol catabolic process",
  "term_id": "GO:0019563",
  "gene": "UniProtKB:Q3LXA3",
  "gene_name": "Triokinase_FMN cyclase"
}